ribonuclease F activity [GO:0033900] (MF) Also known as: RNase F activity, ribonuclease F (E. coli) activity Relationships: is a type of GO:0016892 Sources: EC:3.1.27.7 Definition: Catalysis of the endonucleolytic cleavage of RNA precursor into two, leaving 5'-hydroxy and 3'-phosphate groups.